{
  "gene_name": "Protein LRATD1",
  "gene_symbol": "LRATD1",
  "term_id": "GO:0000902",
  "gene": "UniProtKB:Q96KN4",
  "term_label": "cell morphogenesis"
}